{
  "term_label": "Z disc",
  "term_id": "GO:0030018",
  "gene_name": "LIM domain-binding protein 3",
  "gene_symbol": "LDB3",
  "gene": "UniProtKB:O75112"
}